microglial cell migration [GO:1904124] (biological process) References: PMID:19100238 Sources: GOC:BHF, GOC:TermGenie, GOC:nc, GO_REF:0000091 Relationships: is a type of GO:0008347; is a type of macrophage migration [GO:1905517] Definition: The orderly movement of a microglial cell from one site to another. Regulation: regulated by regulation of microglial cell migration [GO:1904139]; negatively regulated by negative regulation of microglial cell migration [GO:1904140]; positively regulated by positive regulation of microglial cell migration [GO:1904141]